{
  "gene": "UniProtKB:Q15554",
  "gene_name": "Telomeric repeat-binding factor 2",
  "term_label": "telomeric loop formation",
  "gene_symbol": "TERF2",
  "term_id": "GO:0031627"
}